{
  "gene_symbol": "OAS1",
  "gene_name": "2'-5'-oligoadenylate synthase 1",
  "term_id": "GO:0070106",
  "term_label": "interleukin-27-mediated signaling pathway",
  "gene": "UniProtKB:P00973"
}